{
  "term_label": "Unknown biological process",
  "gene_name": "UPF0696 protein C11orf68",
  "term_id": "UNKNOWN:0002",
  "gene": "UniProtKB:Q9H3H3",
  "gene_symbol": "C11orf68"
}